{
  "term_label": "heparan sulfate proteoglycan biosynthetic process",
  "gene": "UniProtKB:Q7LGA3",
  "term_id": "GO:0015012",
  "gene_symbol": "HS2ST1",
  "gene_name": "Heparan sulfate 2-O-sulfotransferase 1"
}